{
  "term_id": "GO:1904315",
  "gene_name": "Glutamate receptor 3",
  "gene_symbol": "GRIA3",
  "gene": "UniProtKB:P42263",
  "term_label": "transmitter-gated monoatomic ion channel activity involved in regulation of postsynaptic membrane potential"
}